{
  "gene_name": "Gamma-aminobutyric acid type B receptor subunit 1",
  "gene_symbol": "GABBR1",
  "gene": "UniProtKB:Q9UBS5",
  "term_label": "G protein-coupled receptor heterodimeric complex",
  "term_id": "GO:0038039"
}